{
  "gene_symbol": "KRT26",
  "term_label": "keratin filament",
  "gene": "UniProtKB:Q7Z3Y9",
  "term_id": "GO:0045095",
  "gene_name": "Keratin, type I cytoskeletal 26"
}